negative regulation of extrinsic apoptotic signaling pathway [GO:2001237] (biological process) Definition: Any process that stops, prevents or reduces the frequency, rate or extent of extrinsic apoptotic signaling pathway. Relationships: is a type of negative regulation of apoptotic signaling pathway [GO:2001234]; is a type of regulation of extrinsic apoptotic signaling pathway [GO:2001236]; negatively regulates extrinsic apoptotic signaling pathway [GO:0097191] Also known as: negative regulation of extrinsic apoptotic signalling pathway, negative regulation of extrinsic apoptosis Sources: GOC:mtg_apoptosis Subtypes: negative regulation of extrinsic apoptotic signaling pathway via death domain receptors [GO:1902042], negative regulation of death-inducing signaling complex assembly [GO:1903073], negative regulation of extrinsic apoptotic signaling pathway in absence of ligand [GO:2001240]